protein transport across the cell outer membrane [GO:0098776] (biological process) Subtypes: protein secretion by the type II secretion system [GO:0015628], protein secretion by the type V secretion system [GO:0046819], protein secretion by the type VIII secretion system [GO:0098777] Sources: GOC:dos Relationships: is a type of protein transmembrane transport [GO:0071806] Definition: The directed movement of proteins across the cell outer membrane.